granulocyte macrophage colony-stimulating factor receptor complex [GO:0030526] (cellular component) Definition: The heterodimeric receptor for granulocyte macrophage colony-stimulating factor. Sources: GOC:mah Relationships: is_a plasma membrane signaling receptor complex [GO:0098802] Also known as: GM-CSF receptor complex, granulocyte macrophage colony stimulating factor receptor complex